{
  "term_label": "nucleus",
  "gene_name": "Zinc finger protein 677",
  "gene_symbol": "ZNF677",
  "gene": "UniProtKB:Q86XU0",
  "term_id": "GO:0005634"
}